{
  "gene": "UniProtKB:Q5D1E8",
  "gene_name": "Endoribonuclease ZC3H12A",
  "gene_symbol": "ZC3H12A",
  "term_label": "RNA endonuclease activity",
  "term_id": "GO:0004521"
}